negative regulation of vascular endothelial cell proliferation [GO:1905563] (biological process) Also known as: down regulation of vascular endothelial cell proliferation, down-regulation of vascular endothelial cell proliferation, downregulation of vascular endothelial cell proliferation, inhibition of vascular endothelial cell proliferation Definition: Any process that stops, prevents or reduces the frequency, rate or extent of vascular endothelial cell proliferation. Relationships: is a type of negative regulation of endothelial cell proliferation [GO:0001937]; is a type of GO:1905562; negatively regulates vascular endothelial cell proliferation [GO:0101023] References: PMID:23201774 Sources: GOC:BHF, GOC:BHF_telomere, GOC:TermGenie, GOC:nc, GO_REF:0000058